{
  "gene_name": "Ribosome biogenesis protein BOP1",
  "gene_symbol": "BOP1",
  "gene": "UniProtKB:Q14137",
  "term_label": "maturation of LSU-rRNA from tricistronic rRNA transcript (SSU-rRNA, 5.8S rRNA, LSU-rRNA)",
  "term_id": "GO:0000463"
}